{
  "gene": "UniProtKB:Q6PL18",
  "term_id": "GO:0042393",
  "gene_symbol": "ATAD2",
  "term_label": "histone binding",
  "gene_name": "ATPase family AAA domain-containing protein 2"
}